leukotriene receptor binding [GO:0031774] (molecular function) Definition: Binding to a leukotriene receptor. Also known as: leukotriene receptor ligand Sources: GOC:mah, GOC:nln Relationships: is a type of GO:0001664